{
  "term_label": "protein K63-linked ubiquitination",
  "term_id": "GO:0070534",
  "gene": "UniProtKB:Q9Y2X8",
  "gene_name": "Ubiquitin-conjugating enzyme E2 D4",
  "gene_symbol": "UBE2D4"
}